{
  "gene_name": "F-box only protein 28",
  "gene": "UniProtKB:Q9NVF7",
  "gene_symbol": "FBXO28",
  "term_label": "Unknown cellular component",
  "term_id": "UNKNOWN:0003"
}